2-octaprenyl-6-methoxyphenol hydroxylase activity [GO:0008681] (molecular function) References: PMID:27822549, PMID:4572721 Sources: RHEA:29407 Relationships: is a type of GO:0016709 Definition: Catalysis of the reaction: 2-methoxy-6-(all-trans-octaprenyl)phenol + H+ + NADPH + O2 = 2-methoxy-6-all-trans-octaprenyl-1,4-benzoquinol + H2O + NADP+.